{
  "term_id": "GO:0005496",
  "gene_symbol": "HSD11B1",
  "gene_name": "11-beta-hydroxysteroid dehydrogenase 1",
  "term_label": "steroid binding",
  "gene": "UniProtKB:P28845"
}